negative regulation of chorionic trophoblast cell proliferation [GO:1901383] (biological process) Definition: Any process that stops, prevents or reduces the frequency, rate or extent of chorionic trophoblast cell proliferation. Sources: GOC:BHF, GOC:TermGenie Also known as: down regulation of chorionic trophoblast cell proliferation, down-regulation of chorionic trophoblast cell proliferation, downregulation of chorionic trophoblast cell proliferation, inhibition of chorionic trophoblast cell proliferation Relationships: is a type of negative regulation of cell population proliferation [GO:0008285]; is a type of regulation of chorionic trophoblast cell proliferation [GO:1901382]; negatively regulates chorionic trophoblast cell proliferation [GO:0097360]